{
  "term_id": "GO:0000226",
  "term_label": "microtubule cytoskeleton organization",
  "gene_symbol": "DYNC1LI2",
  "gene": "UniProtKB:O43237",
  "gene_name": "Cytoplasmic dynein 1 light intermediate chain 2"
}